protein localization to linear element [GO:0036181] (biological process) Also known as: protein localisation to linear element Relationships: is a type of GO:1903084 References: PMID:19756689 Sources: GOC:mah Definition: A cellular protein localization process in which a protein is transported to, or maintained at, a linear element. A linear element is a proteinaceous scaffold associated with S. pombe chromosomes during meiotic prophase.